Nicalin-NOMO complex [GO:0106249] (cellular component) References: PMID:20538592 Sources: GOC:al, GOC:bhm Definition: A protein complex regulating Nodal signaling. Subunits are highly conserved in vertebrates and include Nicalin, NOMO and TMEM147. Relationships: is a type of protein-containing complex [GO:0032991] Also known as: Nicalin-TMEM147-NOMO complex